{
  "gene_symbol": "C1QTNF9B",
  "gene_name": "Complement C1q and tumor necrosis factor-related protein 9B",
  "term_label": "Unknown cellular component",
  "gene": "UniProtKB:B2RNN3",
  "term_id": "UNKNOWN:0003"
}